UTP:galactose-1-phosphate uridylyltransferase activity [GO:0017103] (molecular function) Sources: EC:2.7.7.10, RHEA:14209 Also known as: Gal-1-P uridylyltransferase activity, UTP:hexose-1-phosphate uridylyltransferase activity, galactose-1-phosphate uridylyltransferase activity, UDPgalactose pyrophosphorylase activity, UTP-hexose-1-phosphate uridylyltransferase activity, UTP:alpha-D-hexose-1-phosphate uridylyltransferase activity, alpha-D-galactose 1-phosphate uridylyltransferase activity, galactose 1-phosphate uridyltransferase activity, galactose 1-phosphate uridylyltransferase activity, uridine diphosphate galactose pyrophosphorylase activity, uridine diphosphogalactose pyrophosphorylase activity Relationships: is_a UTP-monosaccharide-1-phosphate uridylyltransferase activity [GO:0051748] Definition: Catalysis of the reaction: alpha-D-galactose 1-phosphate + UTP = diphosphate + UDP-D-galactose.